{
  "gene_name": "Nucleolysin TIAR",
  "gene": "UniProtKB:Q01085",
  "term_id": "GO:0000381",
  "term_label": "regulation of alternative mRNA splicing, via spliceosome",
  "gene_symbol": "TIAL1"
}